{
  "gene_name": "Alanyl-tRNA editing protein Aarsd1",
  "term_label": "Unknown cellular component",
  "gene": "UniProtKB:Q9BTE6",
  "term_id": "UNKNOWN:0003",
  "gene_symbol": "AARSD1"
}